{
  "term_id": "UNKNOWN:0001",
  "gene_name": "Coatomer subunit alpha",
  "term_label": "Unknown molecular function",
  "gene_symbol": "COPA",
  "gene": "UniProtKB:P53621"
}